{
  "gene": "UniProtKB:A0A075B6N1",
  "term_label": "cell surface receptor signaling pathway",
  "term_id": "GO:0007166",
  "gene_symbol": "TRBV19",
  "gene_name": "T cell receptor beta variable 19"
}